{
  "gene_name": "Crossover junction endonuclease MUS81",
  "term_label": "resolution of meiotic recombination intermediates",
  "gene": "UniProtKB:Q96NY9",
  "term_id": "GO:0000712",
  "gene_symbol": "MUS81"
}